{
  "gene_symbol": "POU3F3",
  "term_label": "regulation of transcription by RNA polymerase II",
  "gene": "UniProtKB:P20264",
  "term_id": "GO:0006357",
  "gene_name": "POU domain, class 3, transcription factor 3"
}